{
  "gene": "UniProtKB:P25090",
  "gene_name": "N-formyl peptide receptor 2",
  "term_id": "GO:0004982",
  "term_label": "N-formyl peptide receptor activity",
  "gene_symbol": "FPR2"
}